{
  "term_label": "mesoderm formation",
  "gene_name": "Mesoderm posterior protein 1",
  "gene_symbol": "MESP1",
  "gene": "UniProtKB:Q9BRJ9",
  "term_id": "GO:0001707"
}